cell cortex of non-growing cell tip [GO:0140472] (cellular component) Definition: The region directly beneath the plasma membrane at the cell tip at which no growth takes place. References: PMID:17895368 Relationships: is a type of cell cortex of cell tip [GO:0051285]; is part of non-growing cell tip [GO:0035839]